{
  "gene_name": "Transcription factor COE3",
  "term_label": "Unknown cellular component",
  "gene": "UniProtKB:Q9H4W6",
  "gene_symbol": "EBF3",
  "term_id": "UNKNOWN:0003"
}